chondroitin AC lyase activity [GO:0030341] (molecular function) Sources: EC:4.2.2.5 Definition: Catalysis of the eliminative degradation of polysaccharides containing 1,4-beta-D-hexosaminyl and 1,3-beta-D-glucuronosyl linkages to disaccharides containing 4-deoxy-beta-D-gluc-4-enuronosyl groups. Relationships: is a type of carbon-oxygen lyase activity, acting on polysaccharides [GO:0016837] Also known as: chondroitinase activity, chondroitin lyase activity, ChnAC, chondroitin AC eliminase activity, chondroitin sulfate lyase activity, chondroitinase AC